{
  "term_id": "UNKNOWN:0003",
  "gene_name": "Suppressyn",
  "gene_symbol": "ERVH48-1",
  "term_label": "Unknown cellular component",
  "gene": "UniProtKB:M5A8F1"
}